super elongation complex [GO:0032783] (cellular component) Relationships: is a type of transcription elongation factor complex [GO:0008023] References: PMID:17150956, PMID:30102332 Also known as: ELL-EAF complex, ELL-EAF-EBP complex Definition: A transcription elongation factor complex that increases the overall rate of RNA polymerase II transcription elongation by suppressing transient polymerase pausing. At minimum, the complex contains a transcription factor of the ELL family, an EAF protein, and an AFF family protein or distant relative and most likely also P-TEFb and AF9 or ENL. The complex is conserved from yeast to humans. In Schizosaccharomyces pombe it contains Ell1, Eaf1, and Ebp1, but it is absent from S. cerevisiae.